{
  "gene": "UniProtKB:P78413",
  "term_label": "regulation of transcription by RNA polymerase II",
  "gene_symbol": "IRX4",
  "gene_name": "Iroquois-class homeodomain protein IRX-4",
  "term_id": "GO:0006357"
}